{
  "gene_name": "Putative RNA-binding protein Luc7-like 1",
  "term_id": "GO:0005685",
  "gene_symbol": "LUC7L",
  "term_label": "U1 snRNP",
  "gene": "UniProtKB:Q9NQ29"
}